negative regulation of testosterone biosynthetic process [GO:2000225] (biological process) Definition: Any process that stops, prevents, or reduces the frequency, rate or extent of testosterone biosynthetic process. Sources: GOC:obol, GOC:yaf Relationships: is a type of negative regulation of steroid biosynthetic process [GO:0010894]; is a type of GO:0062014; is_a regulation of testosterone biosynthetic process [GO:2000224]; negatively regulates GO:0061370